{
  "gene_symbol": "CIZ1",
  "term_label": "nucleus",
  "gene_name": "Cip1-interacting zinc finger protein",
  "term_id": "GO:0005634",
  "gene": "UniProtKB:Q9ULV3"
}